{
  "term_id": "GO:0051233",
  "gene_name": "Borealin",
  "gene_symbol": "CDCA8",
  "gene": "UniProtKB:Q53HL2",
  "term_label": "spindle midzone"
}